positive regulation of endoplasmic reticulum tubular network organization [GO:1903373] (biological process) References: PMID:24891604 Sources: GOC:TermGenie, GOC:als, GO_REF:0000058 Definition: Any process that activates or increases the frequency, rate or extent of endoplasmic reticulum tubular network organization. Relationships: is a type of positive regulation of organelle organization [GO:0010638]; is a type of GO:1903371; positively regulates endoplasmic reticulum tubular network organization [GO:0071786] Also known as: positive regulation of ER tubular network organisation, positive regulation of ER tubular network organization, positive regulation of endoplasmic reticulum tubular network organisation, up regulation of ER tubular network organisation, up regulation of ER tubular network organization, up regulation of endoplasmic reticulum tubular network organisation, up regulation of endoplasmic reticulum tubular network organization, up-regulation of ER tubular network organisation, up-regulation of ER tubular network organization, up-regulation of endoplasmic reticulum tubular network organisation, up-regulation of endoplasmic reticulum tubular network organization, upregulation of ER tubular network organisation, upregulation of ER tubular network organization, upregulation of endoplasmic reticulum tubular network organisation, upregulation of endoplasmic reticulum tubular network organization, activation of ER tubular network organisation, activation of ER tubular network organization, activation of endoplasmic reticulum tubular network organisation, activation of endoplasmic reticulum tubular network organization